{
  "gene_name": "Leucine-rich repeat-containing protein 2",
  "gene_symbol": "LRRC2",
  "gene": "UniProtKB:Q9BYS8",
  "term_label": "intracellular signal transduction",
  "term_id": "GO:0035556"
}